stomatal movement [GO:0010118] (biological process) Relationships: is a type of cellular process [GO:0009987] Definition: The process of opening or closing of stomata, which is directly related to the stomatal conductance (measuring rate of passage of either water vapor or carbon dioxide (CO2) through stomata). Subtypes: stomatal closure [GO:0090332], stomatal opening [GO:1990069] Regulation: regulated by regulation of stomatal movement [GO:0010119] Sources: GOC:sm